{
  "term_label": "Unknown cellular component",
  "term_id": "UNKNOWN:0003",
  "gene_symbol": "NWD1",
  "gene_name": "NACHT domain- and WD repeat-containing protein 1",
  "gene": "UniProtKB:Q149M9"
}